response to water-immersion restraint stress [GO:1990785] (biological process) Also known as: response to immobilization stress combined with water immersion Relationships: is_a GO:0035902 Definition: Any process that results in a change in state or activity of a cell or an organism (in terms of movement, secretion, enzyme production, gene expression, etc.) as a result of water immersion while being held immobile. References: PMID:10882227